{
  "gene_name": "Olfactory receptor 52I1",
  "gene_symbol": "OR52I1",
  "gene": "UniProtKB:Q8NGK6",
  "term_label": "olfactory receptor activity",
  "term_id": "GO:0004984"
}